{
  "term_id": "GO:0043161",
  "gene": "UniProtKB:P54727",
  "gene_symbol": "RAD23B",
  "gene_name": "UV excision repair protein RAD23 homolog B",
  "term_label": "proteasome-mediated ubiquitin-dependent protein catabolic process"
}